{
  "gene_name": "Zinc transporter SLC39A7",
  "term_id": "GO:0005385",
  "gene_symbol": "SLC39A7",
  "gene": "UniProtKB:Q92504",
  "term_label": "zinc ion transmembrane transporter activity"
}